{
  "gene": "UniProtKB:Q8TC05",
  "term_label": "retina development in camera-type eye",
  "gene_name": "Nuclear protein MDM1",
  "gene_symbol": "MDM1",
  "term_id": "GO:0060041"
}